peptidyl-lysine glutarylation [GO:0106227] (BP) References: PMID:31542297 Sources: GOC:sp Relationships: is a type of protein acylation [GO:0043543] Definition: The glutarylation of a lysine residue in a protein.